{
  "gene_symbol": "PRSS27",
  "term_id": "GO:0016485",
  "term_label": "protein processing",
  "gene": "UniProtKB:Q9BQR3",
  "gene_name": "Serine protease 27"
}